site-specific DNA-methyltransferase (cytosine-N4-specific) activity [GO:0015667] (molecular function) Relationships: is a type of GO:0008757; is a type of GO:0009008 Definition: Catalysis of the reaction: S-adenosyl-L-methionine + DNA cytosine = S-adenosyl-L-homocysteine + DNA N4-methylcytosine. Also known as: DNA[cytosine-N4]methyltransferase activity, N(4)-cytosine-specific DNA methylase activity, N4-cytosine-specific DNA methylase activity, S-adenosyl-L-methionine:DNA-cytosine 4-N-methyltransferase activity, S-adenosyl-L-methionine:DNA-cytosine N4-methyltransferase activity, m4C-forming MTase activity, modification methylase activity, restriction-modification system activity Sources: EC:2.1.1.113